cyclic-di-GMP transmembrane transporter activity [GO:0140927] (molecular function) References: PMID:34965418 Relationships: is a type of guanine nucleotide transmembrane transporter activity [GO:0001409]; is a type of GO:0005346 Definition: Enables the transfer of cyclic-di-GMP from one side of a membrane to the other.